{
  "term_label": "anterior/posterior pattern specification",
  "gene": "UniProtKB:Q5TA89",
  "term_id": "GO:0009952",
  "gene_name": "Transcription factor HES-5",
  "gene_symbol": "HES5"
}